{
  "gene_name": "Ras-GEF domain-containing family member 1A",
  "term_label": "Ras protein signal transduction",
  "gene": "UniProtKB:Q8N9B8",
  "gene_symbol": "RASGEF1A",
  "term_id": "GO:0007265"
}